negative regulation of endothelial cell activation [GO:1904988] (BP) Definition: Any process that stops, prevents or reduces the frequency, rate or extent of endothelial cell activation. References: PMID:24255059 Sources: GOC:BHF, GOC:BHF_miRNA, GOC:TermGenie, GOC:bc, GO_REF:0000058 Also known as: down regulation of endothelial cell activation, down-regulation of endothelial cell activation, downregulation of endothelial cell activation, inhibition of endothelial cell activation Relationships: is a type of negative regulation of cell activation [GO:0050866]; is a type of regulation of endothelial cell activation [GO:1904987]; negatively regulates endothelial cell activation [GO:0042118]